{
  "term_label": "precatalytic spliceosome",
  "gene_symbol": "PRPF31",
  "gene": "UniProtKB:Q8WWY3",
  "gene_name": "U4_U6 small nuclear ribonucleoprotein Prp31",
  "term_id": "GO:0071011"
}